{
  "term_label": "succinate transmembrane transport",
  "term_id": "GO:0071422",
  "gene_name": "Mitochondrial dicarboxylate carrier",
  "gene_symbol": "SLC25A10",
  "gene": "UniProtKB:Q9UBX3"
}